bacterial-type EF-P lysine modification [GO:0072580] (biological process) References: PMID:20729861, PMID:22706199 Sources: GOC:curators, GOC:imk, GOC:mah, RESID:AA0530, RESID:AA0531 Definition: The modification of a lysine residue in a protein to produce (2S)-2-amino-6-([(3S)-3,6-diaminohexanoyl]amino)hexanoic acid, and the subsequent hydroxylation of the modified lysine residue. This modification is observed in, and is probably unique to, the prokaryotic translation elongation factor P (EF-P). Relationships: is a type of GO:0018205 Note: The EF-P modification pathway is now thought to be composed of three steps: conversion of alpha-lysyl-EF-P to beta-lysyl-EF-P, lysylation of Lys34, and hydroxylation of Lys34. Also known as: EF-P modification pathway